{
  "term_id": "GO:0000785",
  "gene": "UniProtKB:Q9UPN9",
  "gene_name": "E3 ubiquitin-protein ligase TRIM33",
  "gene_symbol": "TRIM33",
  "term_label": "chromatin"
}